regulation of elastin catabolic process [GO:0060310] (biological process) Subtypes: GO:0060311, GO:0110015 Definition: Any process that modulates the rate, frequency or extent of elastin catabolism, the chemical reactions and pathways resulting in the breakdown of elastin. Relationships: is a type of GO:0042176; is a type of regulation of glycoprotein metabolic process [GO:1903018]; regulates elastin catabolic process [GO:0060309] Also known as: regulation of elastin catabolism, regulation of elastin degradation, regulation of elastin breakdown Sources: GOC:BHF, GOC:dph, GOC:tb